positive regulation of appetite [GO:0032100] (biological process) Relationships: is a type of positive regulation of response to food [GO:0032097]; is a type of regulation of appetite [GO:0032098] Definition: Any process that increases appetite. Also known as: up regulation of appetite, up-regulation of appetite, upregulation of appetite, activation of appetite, stimulation of appetite, appetite stimulation, positive regulation of hunger Sources: GOC:add